{
  "term_label": "Unknown molecular function",
  "gene_name": "28S rRNA (cytosine-C(5))-methyltransferase",
  "gene": "UniProtKB:Q96P11",
  "term_id": "UNKNOWN:0001",
  "gene_symbol": "NSUN5"
}